lateral semicircular canal development [GO:0060875] (biological process) Relationships: is a type of GO:0060872 Definition: The progession of the lateral semicircular canal from its initial formation to the mature structure. Sources: GOC:dph, GOC:sdb_2009, GOC:tb